His-Purkinje system cell development [GO:0060933] (biological process) Definition: The process whose specific outcome is the progression of a His-Purkinje cell over time, from its formation to the mature state. These cells form the fibers that regulate cardiac muscle contraction in the ventricles. Sources: GOC:mtg_heart Relationships: is a type of cardiac cell development [GO:0055006]; is part of His-Purkinje system cell differentiation [GO:0060932]